averantin catabolic process [GO:1900762] (biological process) Definition: The chemical reactions and pathways resulting in the breakdown of averantin. Sources: GOC:TermGenie, GOC:di Also known as: averantin breakdown, averantin catabolism, averantin degradation Relationships: is_a phenol-containing compound catabolic process [GO:0019336]; is a type of polyketide catabolic process [GO:0030640]; is_a ketone catabolic process [GO:0042182]